regulation of establishment of bipolar cell polarity [GO:0061172] (BP) Sources: GOC:dph, GOC:vw Definition: Any process that modulates the rate, frequency or extent of the establishment of bipolar cell polarity. Bipolar organization is the organization that is a mirror image along an axis from a plane. Relationships: is a type of regulation of establishment of cell polarity [GO:2000114]; regulates establishment of bipolar cell polarity [GO:0061171] Subtypes: regulation of establishment of bipolar cell polarity regulating cell shape [GO:0061160], positive regulation of establishment of bipolar cell polarity [GO:0061173], negative regulation of establishment of bipolar cell polarity [GO:1904846]